calcium:proton antiporter complex [GO:0061993] (cellular component) Also known as: CAX1 homodimer, CAX1-CAX3 complex, CAX3 homodimer Relationships: is_a transmembrane transporter complex [GO:1902495] References: PMID:19098009, PMID:28645169 Sources: GOC:bhm Definition: A protein complex that enables the transfer of a solute or solutes from one side of a membrane to the other according to the reaction: Ca2+(in) + H+(out) = Ca2+(out) + H+(in).